{
  "term_id": "UNKNOWN:0001",
  "gene_symbol": "PNMA6F",
  "gene_name": "Paraneoplastic antigen Ma6F",
  "gene": "UniProtKB:A0A0J9YX94",
  "term_label": "Unknown molecular function"
}